{
  "gene_name": "TYMS opposite strand protein",
  "gene_symbol": "TYMSOS",
  "gene": "UniProtKB:Q8TAI1",
  "term_id": "UNKNOWN:0001",
  "term_label": "Unknown molecular function"
}